{
  "gene_name": "Fermitin family homolog 2",
  "gene": "UniProtKB:Q96AC1",
  "term_id": "GO:0007160",
  "term_label": "cell-matrix adhesion",
  "gene_symbol": "FERMT2"
}